{
  "gene_name": "Ciliary neurotrophic factor",
  "gene_symbol": "CNTF",
  "term_label": "cytokine activity",
  "gene": "UniProtKB:P26441",
  "term_id": "GO:0005125"
}